regulation of stem cell division [GO:2000035] (biological process) Relationships: is a type of regulation of cell division [GO:0051302]; regulates GO:0017145 Subtypes: regulation of somatic stem cell division [GO:1904675], regulation of male germ-line stem cell asymmetric division [GO:1904838] Also known as: regulation of stem cell renewal Sources: GOC:obol Definition: Any process that modulates the frequency, rate or extent of stem cell division.